{
  "term_id": "GO:0042742",
  "gene": "UniProtKB:Q13075",
  "term_label": "defense response to bacterium",
  "gene_symbol": "NAIP",
  "gene_name": "Baculoviral IAP repeat-containing protein 1"
}